{
  "gene": "UniProtKB:O43617",
  "gene_name": "Trafficking protein particle complex subunit 3",
  "gene_symbol": "TRAPPC3",
  "term_label": "cis-Golgi network membrane",
  "term_id": "GO:0033106"
}